regulation of isoprenoid metabolic process [GO:0019747] (biological process) Subtypes: regulation of juvenile hormone biosynthetic process [GO:0007557], GO:0010115, regulation of isopentenyl diphosphate biosynthetic process, methylerythritol 4-phosphate pathway [GO:0010322], regulation of gibberellin biosynthetic process [GO:0010371], negative regulation of isoprenoid metabolic process [GO:0045827], GO:0045952, regulation of retinoic acid biosynthetic process [GO:1900052], regulation of isoprene biosynthetic process [GO:1900947], GO:1901542, regulation of vitamin A metabolic process [GO:1901738], positive regulation of carotenoid biosynthetic process [GO:1904143], regulation of phytol biosynthetic process [GO:1904963], regulation of isopentenyl diphosphate biosynthetic process, mevalonate pathway [GO:2001210] Sources: GOC:go_curators Relationships: is a type of GO:0019216; regulates isoprenoid metabolic process [GO:0006720] Definition: Any process that modulates the frequency, rate or extent of the chemical reactions and pathways involving isoprenoids. Also known as: regulation of isoprenoid metabolism